3,4-dichlorobenzoate-4,5-oxygenase activity [GO:0102046] (molecular function) References: PMID:9322760 Sources: GOC:pz Definition: Catalysis of the reaction: 3,4-dichlorobenzoate + O2 + a reduced electron acceptor = 3,4-dichlorobenzoate-cis-4,5-diol + an oxidized electron acceptor. Relationships: is a type of oxidoreductase activity, acting on paired donors, with incorporation or reduction of molecular oxygen, NAD(P)H as one donor, and incorporation of two atoms of oxygen into one donor [GO:0016708]